symbiont-mediated perturbation of host MAPK cascade [GO:0052080] (biological process) Definition: A process in which a symbiont alters or subverts a MAP kinase-mediated signal transduction pathway in its host organism. The host is defined as the larger of the organisms involved in a symbiotic interaction. Sources: GOC:mtg_pamgo_17jul06 Also known as: perturbation by symbiont of host MAP kinase signal transduction pathway, perturbation of host MAP signal transduction pathway, perturbation of host MAPK kinase signaling pathway, perturbation of host MAPK signal transduction pathway, modulation by symbiont of host innate immune response MAPK kinase signaling, modulation of defense-related host MAPK-mediated signal transduction pathway by organism, modulation of defense-related host mitogen activated protein kinase-mediated signal transduction pathway by organism, perturbation of host innate immune response MAPK kinase signaling, modulation by symbiont of defense-related host MAP kinase-mediated signal transduction pathway Relationships: is a type of symbiont-mediated perturbation of host signal transduction pathway [GO:0052027] Subtypes: symbiont-mediated suppression of host MAPK cascade [GO:0141070], symbiont-mediated activation of host MAPK cascade [GO:0141071]